{
  "term_id": "UNKNOWN:0001",
  "gene_name": "Lens fiber membrane intrinsic protein",
  "gene_symbol": "LIM2",
  "term_label": "Unknown molecular function",
  "gene": "UniProtKB:P55344"
}